{
  "term_id": "GO:0003779",
  "term_label": "actin binding",
  "gene_symbol": "NCALD",
  "gene": "UniProtKB:P61601",
  "gene_name": "Neurocalcin-delta"
}